adenylyl-sulfate reductase activity [GO:0009973] (molecular function) Definition: Catalysis of the reaction: A + AMP + 2 H+ + sulfite = adenosine 5'-phosphosulfate + AH2. Also known as: APS reductase activity, adenosine phosphosulfate reductase activity, adenylyl-sulphate reductase activity References: PMID:5421934 Sources: RHEA:24240 Relationships: is a type of GO:0016667